phosphatidylglycerol phospholipase C activity [GO:0034479] (molecular function) Definition: Catalysis of the reaction: a phosphatidylglycerol + H2O = 1,2-diacylglycerol + glycerol 3-phosphate. References: PMID:18434318 Sources: GOC:mah Relationships: is_a GO:0004629